{
  "gene_symbol": "SMPD2",
  "term_id": "GO:0005783",
  "term_label": "endoplasmic reticulum",
  "gene": "UniProtKB:O60906",
  "gene_name": "Sphingomyelin phosphodiesterase 2"
}